{
  "term_label": "extracellular matrix organization",
  "gene_symbol": "SPINT1",
  "gene": "UniProtKB:O43278",
  "gene_name": "Kunitz-type protease inhibitor 1",
  "term_id": "GO:0030198"
}